{
  "term_id": "GO:0071805",
  "gene_symbol": "KCNV2",
  "term_label": "potassium ion transmembrane transport",
  "gene": "UniProtKB:Q8TDN2",
  "gene_name": "Potassium voltage-gated channel subfamily V member 2"
}